tolerance induction in urogenital tract [GO:0002425] (BP) Definition: Tolerance induction taking place in the urogenital tract. Sources: GOC:jal Relationships: is a type of mucosal tolerance induction [GO:0002427]